{
  "gene": "UniProtKB:O95433",
  "gene_name": "Activator of 90 kDa heat shock protein ATPase homolog 1",
  "term_id": "GO:0006457",
  "term_label": "protein folding",
  "gene_symbol": "AHSA1"
}